{
  "gene_symbol": "C1orf162",
  "term_label": "Unknown biological process",
  "gene_name": "Transmembrane protein C1orf162",
  "term_id": "UNKNOWN:0002",
  "gene": "UniProtKB:Q8NEQ5"
}